{
  "term_label": "extracellular space",
  "gene_name": "Left-right determination factor 2",
  "gene": "UniProtKB:O00292",
  "gene_symbol": "LEFTY2",
  "term_id": "GO:0005615"
}